{
  "gene": "UniProtKB:Q8N5Z0",
  "gene_name": "Kynurenine_alpha-aminoadipate aminotransferase, mitochondrial",
  "term_label": "alpha-amino acid metabolic process",
  "term_id": "GO:1901605",
  "gene_symbol": "AADAT"
}